{
  "term_id": "GO:0007286",
  "gene_symbol": "RFX2",
  "gene_name": "DNA-binding protein RFX2",
  "term_label": "spermatid development",
  "gene": "UniProtKB:P48378"
}